{
  "term_id": "GO:0033204",
  "gene_symbol": "POP4",
  "gene_name": "Ribonuclease P protein subunit p29",
  "term_label": "ribonuclease P RNA binding",
  "gene": "UniProtKB:O95707"
}